{
  "gene": "UniProtKB:A8MV57",
  "gene_name": "Putative mucosal pentraxin homolog",
  "term_label": "Unknown biological process",
  "term_id": "UNKNOWN:0002",
  "gene_symbol": "MPTX1"
}